intestinal epithelial structure maintenance [GO:0060729] (biological process) Also known as: epithelial structure maintenance of intestine, maintenance of intestinal epithelium Sources: GOC:BHF, GOC:dph, GOC:tb Regulation: regulated by regulation of intestinal epithelial structure maintenance [GO:0060730]; positively regulated by positive regulation of intestinal epithelial structure maintenance [GO:0060731] Relationships: is a type of maintenance of gastrointestinal epithelium [GO:0030277] Definition: A tissue homeostatic process required for the maintenance of the structure of the intestinal epithelium.